positive regulation of apoptotic process [GO:0043065] (biological process) Also known as: up regulation of apoptosis, up-regulation of apoptosis, upregulation of apoptosis, activation of apoptosis, positive regulation of apoptosis, stimulation of apoptosis, pro-apoptosis Sources: GOC:jl, GOC:mtg_apoptosis Definition: Any process that activates or increases the frequency, rate or extent of cell death by apoptotic process. Subtypes: GO:0010661, positive regulation of myeloid cell apoptotic process [GO:0033034], positive regulation of glial cell apoptotic process [GO:0034352], positive regulation of neuron apoptotic process [GO:0043525], positive regulation of apoptotic process in bone marrow cell [GO:0120132], GO:1900119, positive regulation of compound eye retinal cell apoptotic process [GO:1901694], GO:1904037, positive regulation of myofibroblast cell apoptotic process [GO:1904522], positive regulation of fat cell apoptotic process [GO:1904651], positive regulation of apoptotic process involved in development [GO:1904747], positive regulation of leukocyte apoptotic process [GO:2000108], GO:2000210, positive regulation of fibroblast apoptotic process [GO:2000271], positive regulation of endothelial cell apoptotic process [GO:2000353], GO:2001055, positive regulation of apoptotic signaling pathway [GO:2001235] Note: This term should only be used when it is not possible to determine which phase or subtype of the apoptotic process is positively regulated by a gene product. Whenever detailed information is available, the more granular children terms should be used. Relationships: is a type of regulation of apoptotic process [GO:0042981]; is a type of positive regulation of programmed cell death [GO:0043068]; positively regulates apoptotic process [GO:0006915]